{
  "gene_symbol": "ZFP64",
  "gene": "UniProtKB:Q9NTW7",
  "term_label": "DNA-binding transcription factor activity",
  "term_id": "GO:0003700",
  "gene_name": "Zinc finger protein 64"
}